{
  "term_id": "GO:0051087",
  "gene": "UniProtKB:Q8WW22",
  "term_label": "protein-folding chaperone binding",
  "gene_symbol": "DNAJA4",
  "gene_name": "DnaJ homolog subfamily A member 4"
}